{
  "gene_symbol": "GBP7",
  "term_id": "GO:0042832",
  "gene": "UniProtKB:Q8N8V2",
  "gene_name": "Guanylate-binding protein 7",
  "term_label": "defense response to protozoan"
}